{
  "term_id": "GO:0007159",
  "gene": "UniProtKB:P05107",
  "gene_name": "Integrin beta-2",
  "gene_symbol": "ITGB2",
  "term_label": "leukocyte cell-cell adhesion"
}